{
  "gene_name": "Nucleolar protein 12",
  "gene": "UniProtKB:Q9UGY1",
  "term_label": "rRNA binding",
  "gene_symbol": "NOL12",
  "term_id": "GO:0019843"
}